{
  "term_id": "GO:0034727",
  "gene_name": "Sorting nexin-30",
  "gene_symbol": "SNX30",
  "term_label": "piecemeal microautophagy of the nucleus",
  "gene": "UniProtKB:Q5VWJ9"
}